{
  "term_label": "negative regulation of Notch signaling pathway",
  "gene_name": "Transcriptional and immune response regulator",
  "gene_symbol": "TCIM",
  "gene": "UniProtKB:Q9NR00",
  "term_id": "GO:0045746"
}